regulation of induction of conjugation upon nitrogen starvation [GO:0060905] (biological process) Sources: GOC:dph, GOC:tb Relationships: is a type of regulation of conjugation with cellular fusion [GO:0031137]; is_a regulation of response to nutrient levels [GO:0032107]; is a type of regulation of cellular response to stress [GO:0080135]; regulates induction of conjugation upon nitrogen starvation [GO:0031142] Definition: Any process that modulates the frequency of induction of conjugation upon nitrogen starvation, the process in which a cell initiates conjugation with cellular fusion upon nitrogen starvation.